{
  "term_id": "GO:0097623",
  "gene_symbol": "KCND3",
  "gene": "UniProtKB:Q9UK17",
  "term_label": "potassium ion export across plasma membrane",
  "gene_name": "Potassium voltage-gated channel subfamily D member 3"
}